dosage compensation by hypoactivation of X chromosome [GO:0042464] (biological process) Definition: Compensating for the two-fold variation in X:autosome chromosome ratios between sexes by an inactivation of a proportion of genes on both of the X chromosomes of the XX sex, leading to a decrease, of half, of the levels of gene expression from these chromosomes. An example of this process is found in Caenorhabditis elegans. Relationships: is a type of sex-chromosome dosage compensation [GO:0007549] References: PMID:11102361 Sources: GOC:jl, GOC:mr